{
  "gene": "UniProtKB:Q99959",
  "term_id": "GO:0072659",
  "term_label": "protein localization to plasma membrane",
  "gene_name": "Plakophilin-2",
  "gene_symbol": "PKP2"
}